{
  "term_label": "Unknown cellular component",
  "gene_name": "L-amino-acid oxidase",
  "term_id": "UNKNOWN:0003",
  "gene": "UniProtKB:Q96RQ9",
  "gene_symbol": "IL4I1"
}